ergothioneine biosynthesis from histidine via gamma-glutamyl-hercynylcysteine sulfoxide [GO:0052704] (BP) References: PMID:4276459, PMID:5484456 Also known as: ergothioneine biosynthesis from histidine via N-alpha,N-alpha,N-alpha-trimethyl-L-histidine Definition: The pathway resulting in the formation of ergothioneine from histidine via a set of steps in which gamma-glutamyl-hercynylcysteine sulfoxide is formed as an intermediate. Relationships: is a type of ergothioneine biosynthetic process [GO:0052699]